{
  "term_label": "nucleus",
  "gene_name": "Gem-associated protein 5",
  "gene_symbol": "GEMIN5",
  "term_id": "GO:0005634",
  "gene": "UniProtKB:Q8TEQ6"
}